response to formaldehyde [GO:1904404] (biological process) Definition: Any process that results in a change in state or activity of a cell or an organism (in terms of movement, secretion, enzyme production, gene expression, etc.) as a result of a formaldehyde stimulus. References: PMID:9149109 Sources: GOC:TermGenie, GO_REF:0000071 Relationships: is a type of GO:1901700 Subtypes: GO:1904405